{
  "term_label": "lysosome localization",
  "gene": "UniProtKB:Q96GS4",
  "gene_name": "BLOC-1-related complex subunit 6",
  "gene_symbol": "BORCS6",
  "term_id": "GO:0032418"
}